{
  "gene_symbol": "RCSD1",
  "gene_name": "CapZ-interacting protein",
  "gene": "UniProtKB:Q6JBY9",
  "term_label": "early endosome",
  "term_id": "GO:0005769"
}